glycyrrhetinate catabolic process [GO:1902385] (BP) Definition: The chemical reactions and pathways resulting in the breakdown of glycyrrhetinate. Also known as: glycyrrhetinate breakdown, glycyrrhetinate catabolism, glycyrrhetinate degradation Relationships: is a type of pentacyclic triterpenoid catabolic process [GO:0019741]; is a type of ketone catabolic process [GO:0042182]; is a type of monocarboxylic acid catabolic process [GO:0072329] References: PMID:22128119 Sources: GOC:TermGenie